{
  "gene_name": "Transmembrane emp24 domain-containing protein 10",
  "gene_symbol": "TMED10",
  "term_id": "GO:0007030",
  "term_label": "Golgi organization",
  "gene": "UniProtKB:P49755"
}